{
  "gene_symbol": "SNAP25",
  "gene_name": "Synaptosomal-associated protein 25",
  "term_id": "GO:0016082",
  "gene": "UniProtKB:P60880",
  "term_label": "synaptic vesicle priming"
}